endolysosome [GO:0036019] (cellular component) References: PMID:21878991 Sources: GOC:pde Relationships: is a type of lysosome [GO:0005764]; is a type of endosome [GO:0005768] Definition: An transient hybrid organelle formed by fusion of a late endosome with a lysosome, and in which active degradation takes place.